{
  "gene": "UniProtKB:Q99569",
  "term_id": "GO:0005634",
  "gene_name": "Plakophilin-4",
  "gene_symbol": "PKP4",
  "term_label": "nucleus"
}